{
  "term_label": "neuronal cell body",
  "term_id": "GO:0043025",
  "gene_name": "Ciliary neurotrophic factor",
  "gene": "UniProtKB:P26441",
  "gene_symbol": "CNTF"
}